myoblast fusion involved in skeletal muscle regeneration [GO:0014905] (biological process) Sources: CL:0000056, GOC:mtg_muscle Definition: A process in which non-proliferating myoblasts, after migrating to the site of injury, fuse into existing damaged fibers or fuse to myotubes to form new fibers, as part of the process of skeletal muscle regeneration. A myoblast is a mononucleate cell type that, by fusion with other myoblasts, gives rise to the myotubes that eventually develop into skeletal muscle fibers. Relationships: is a type of myoblast fusion [GO:0007520]; is part of myotube differentiation involved in skeletal muscle regeneration [GO:0014908]